CUG codon-amino acid adaptor activity [GO:0033420] (molecular function) Definition: A triplet codon-amino acid adaptor activity that recognizes a CUG codon. Note: Note that in the standard genetic code, CTG codes for leucine. Sources: GOC:mah Also known as: CTG codon-amino acid adaptor activity, leucine tRNA Relationships: is a type of GO:0030533